chemorepellent activity [GO:0045499] (molecular function) Relationships: is a type of GO:0048018; is part of negative chemotaxis [GO:0050919] Sources: GOC:ai Also known as: chemorepellant activity Definition: Providing the environmental signal that initiates the directed movement of a motile cell or organism towards a lower concentration of that signal.